{
  "gene_symbol": "CNTNAP2",
  "gene_name": "Contactin-associated protein-like 2",
  "term_label": "synapse",
  "gene": "UniProtKB:Q9UHC6",
  "term_id": "GO:0045202"
}